{
  "term_label": "induction of positive chemotaxis",
  "gene_name": "Placenta growth factor",
  "gene": "UniProtKB:P49763",
  "gene_symbol": "PGF",
  "term_id": "GO:0050930"
}